regulation of calcium ion import across plasma membrane [GO:1905664] (biological process) Relationships: is a type of regulation of calcium ion import [GO:0090279]; is a type of regulation of calcium ion transmembrane transport [GO:1903169]; RO_0002211 calcium ion import across plasma membrane [GO:0098703] Definition: Any process that modulates the frequency, rate or extent of calcium ion import across plasma membrane. References: PMID:17640527 Sources: GOC:TermGenie, GOC:bhm, GO_REF:0000058 Subtypes: positive regulation of calcium ion import across plasma membrane [GO:1905665], GO:1905949 Note: An example of this is PPP3CA in human (Q08209) in 17640527 (inferred from direct assay).